{
  "term_label": "G2/M transition of mitotic cell cycle",
  "gene": "UniProtKB:Q00534",
  "gene_symbol": "CDK6",
  "term_id": "GO:0000086",
  "gene_name": "Cyclin-dependent kinase 6"
}